{
  "gene": "UniProtKB:Q6ZMY6",
  "gene_symbol": "WDR88",
  "term_id": "UNKNOWN:0003",
  "gene_name": "WD repeat-containing protein 88",
  "term_label": "Unknown cellular component"
}